{
  "gene_name": "G-protein coupled receptor 42",
  "gene_symbol": "GPR42",
  "term_label": "Unknown molecular function",
  "term_id": "UNKNOWN:0001",
  "gene": "UniProtKB:O15529"
}